{
  "gene": "UniProtKB:Q9C0A6",
  "gene_symbol": "SETD5",
  "term_id": "GO:0006355",
  "gene_name": "Histone-lysine N-methyltransferase SETD5",
  "term_label": "regulation of DNA-templated transcription"
}